negative regulation of xanthophore differentiation [GO:0050944] (biological process) Sources: GOC:ai Note: Note that this term refers to xanthophores in the sense of specialized pigment-producing cells, and should not be confused with the cellular component term 'xanthophore ; GO:0031633', which refers to a subcellular structure. Also known as: down regulation of xanthophore differentiation, down-regulation of xanthophore differentiation, downregulation of xanthophore differentiation, inhibition of xanthophore differentiation Relationships: is_a regulation of xanthophore differentiation [GO:0050938]; is a type of negative regulation of pigment cell differentiation [GO:0050941]; negatively regulates xanthophore differentiation [GO:0050936] Definition: Any process that stops, prevents, or reduces the frequency, rate or extent of xanthophore differentiation.